{
  "gene": "UniProtKB:Q71UI9",
  "gene_name": "Histone H2A.V",
  "term_label": "nucleus",
  "gene_symbol": "H2AZ2",
  "term_id": "GO:0005634"
}